aerenchyma formation [GO:0010618] (biological process) Definition: The process that gives rise to aerenchyma, parenchyma tissue containing particularly large intercellular spaces of schizogenous or lysigenous origin. This process pertains to the initial formation of a structure from unspecified parts. References: PMID:18055613 Sources: PO:0005702 Relationships: is_a anatomical structure formation involved in morphogenesis [GO:0048646]